{
  "gene_symbol": "LRP5",
  "gene_name": "Low-density lipoprotein receptor-related protein 5",
  "gene": "UniProtKB:O75197",
  "term_label": "nervous system development",
  "term_id": "GO:0007399"
}